{
  "gene_symbol": "MLYCD",
  "term_label": "fatty acid biosynthetic process",
  "term_id": "GO:0006633",
  "gene": "UniProtKB:O95822",
  "gene_name": "Malonyl-CoA decarboxylase, mitochondrial"
}